very long-chain-3-hydroxyacyl-CoA dehydrogenase activity [GO:0035380] (molecular function) Sources: GOC:pde Definition: Catalysis of the reaction: (S)-3-hydroxyacyl-CoA + NAD(P)+ = 3-oxoacyl-CoA + NAD(P)H + H+, where the acyl group is a very long-chain fatty acid residue. A very long-chain fatty acid has an aliphatic tail containing more than 22 carbons. Note: While there is not universal consensus on the lengths of short-, medium-, long- and very-long-chain fatty acids, the GO uses the definitions in ChEBI (see CHEBI:26666, CHEBI:59554, CHEBI:15904 and CHEBI:27283). Relationships: is a type of oxidoreductase activity, acting on the CH-OH group of donors, NAD or NADP as acceptor [GO:0016616] Also known as: very-long-chain-3-hydroxyacyl-CoA dehydrogenase activity